{
  "gene_name": "Protein NPAT",
  "gene_symbol": "NPAT",
  "term_label": "nucleus",
  "gene": "UniProtKB:Q14207",
  "term_id": "GO:0005634"
}